{
  "gene_symbol": "FAM3C",
  "term_label": "signal transduction",
  "term_id": "GO:0007165",
  "gene_name": "Protein FAM3C",
  "gene": "UniProtKB:Q92520"
}